{
  "term_id": "GO:0006357",
  "term_label": "regulation of transcription by RNA polymerase II",
  "gene_name": "Homeobox even-skipped homolog protein 1",
  "gene": "UniProtKB:P49640",
  "gene_symbol": "EVX1"
}